{
  "gene": "UniProtKB:Q15555",
  "gene_name": "Microtubule-associated protein RP_EB family member 2",
  "term_id": "GO:0005881",
  "term_label": "cytoplasmic microtubule",
  "gene_symbol": "MAPRE2"
}